{
  "gene_symbol": "ISY1",
  "term_id": "GO:0071014",
  "term_label": "post-mRNA release spliceosomal complex",
  "gene": "UniProtKB:Q9ULR0",
  "gene_name": "Pre-mRNA-splicing factor ISY1 homolog"
}